radial glial cell division in pallium [GO:0022015] (biological process) Sources: GOC:cls, GOC:dgh, GOC:dph, GOC:jid, GO_REF:0000021 Definition: The division of a radial glial cell in the pallium. A radial glial cell is a precursor cell that gives rise to neurons and astrocytes. Relationships: is a type of cell division [GO:0051301]; is part of pallium cell proliferation in forebrain [GO:0022013]